{
  "gene": "UniProtKB:Q3SYB3",
  "term_id": "GO:0000978",
  "gene_symbol": "FOXD4L6",
  "gene_name": "Forkhead box protein D4-like 6",
  "term_label": "RNA polymerase II cis-regulatory region sequence-specific DNA binding"
}